{
  "gene_symbol": "PIK3CD",
  "term_id": "GO:0043491",
  "gene": "UniProtKB:O00329",
  "term_label": "phosphatidylinositol 3-kinase/protein kinase B signal transduction",
  "gene_name": "Phosphatidylinositol 4,5-bisphosphate 3-kinase catalytic subunit delta isoform"
}